monoatomic ion transmembrane transport [GO:0034220] (biological process) Also known as: ion transmembrane transport, ion membrane transport, transmembrane ion transport, ATP hydrolysis coupled ion transmembrane transport Regulation: regulated by regulation of monoatomic ion transmembrane transport [GO:0034765]; negatively regulated by negative regulation of monoatomic ion transmembrane transport [GO:0034766]; positively regulated by GO:0034767 Sources: GOC:mah Definition: A process in which a monoatomic ion is transported across a membrane. Monatomic ions (also called simple ions) are ions consisting of exactly one atom. Note: Note that this term is not intended for use in annotating lateral movement within membranes. Relationships: is a type of GO:0006811; is a type of transmembrane transport [GO:0055085] Subtypes: establishment or maintenance of transmembrane electrochemical gradient [GO:0010248], monoatomic cation transmembrane transport [GO:0098655], monoatomic anion transmembrane transport [GO:0098656]